{
  "gene_symbol": "BRI3BP",
  "term_label": "Unknown molecular function",
  "term_id": "UNKNOWN:0001",
  "gene": "UniProtKB:Q8WY22",
  "gene_name": "BRI3-binding protein"
}